{
  "term_id": "GO:0007608",
  "gene": "UniProtKB:Q96R08",
  "term_label": "sensory perception of smell",
  "gene_symbol": "OR5B12",
  "gene_name": "Olfactory receptor 5B12"
}